5-alpha-hydroxysteroid dehydratase activity [GO:0047587] (molecular function) Also known as: 5alpha-ergosta-7,22-diene-3beta,5-diol 5,6-hydro-lyase (ergosterol-forming), 5alpha-ergosta-7,22-diene-3beta,5-diol 5,6-hydro-lyase activity, 5alpha-hydroxysteroid dehydratase activity Definition: Catalysis of the reaction: 5alpha-ergosta-7,22-diene-3beta,5-diol = ergosterol + H2O. Sources: EC:4.2.1.62, RHEA:22064 Relationships: is a type of hydro-lyase activity [GO:0016836]